{
  "term_label": "potassium ion transmembrane transport",
  "term_id": "GO:0071805",
  "gene": "UniProtKB:Q9UL51",
  "gene_symbol": "HCN2",
  "gene_name": "Potassium_sodium hyperpolarization-activated cyclic nucleotide-gated channel 2"
}